{
  "term_label": "beta-catenin binding",
  "gene_symbol": "CDH7",
  "gene": "UniProtKB:Q9ULB5",
  "gene_name": "Cadherin-7",
  "term_id": "GO:0008013"
}